{
  "gene_symbol": "NT5C",
  "gene": "UniProtKB:Q8TCD5",
  "gene_name": "5'(3')-deoxyribonucleotidase, cytosolic type",
  "term_label": "pyrimidine deoxyribonucleotide catabolic process",
  "term_id": "GO:0009223"
}